{
  "gene": "UniProtKB:P59022",
  "term_label": "Unknown cellular component",
  "gene_name": "Down syndrome critical region protein 10",
  "gene_symbol": "DSCR10",
  "term_id": "UNKNOWN:0003"
}